metal-dependent deubiquitinase activity [GO:0140492] (molecular function) Relationships: is a type of metallopeptidase activity [GO:0008237]; is a type of deubiquitinase activity [GO:0101005] Also known as: metal-dependent ubiquitin-like hydrolase activity, metal-dependent ubiquitinyl-like hydrolase activity Definition: An metal-dependent isopeptidase activity that cleaves ubiquitin from a target protein to which it is conjugated. References: PMID:19489724